sarcoplasmic reticulum [GO:0016529] (cellular component) Note: See also the cellular component terms 'sarcoplasm ; GO:0016528', 'nuclear envelope ; GO:0005635' and 'endoplasmic reticulum ; GO:0005783'. Relationships: is a type of endoplasmic reticulum [GO:0005783]; is part of sarcoplasm [GO:0016528] Definition: A fine reticular network of membrane-limited elements that pervades the sarcoplasm of a muscle cell; continuous over large portions of the cell and with the nuclear envelope; that part of the endoplasmic reticulum specialized for calcium release, uptake and storage. Sources: GOC:mtg_muscle, ISBN:0124325653, ISBN:0198547684